antifreeze activity [GO:0016172] (MF) Relationships: is a type of ice binding [GO:0050825] Note: Note that this term was reinstated from obsolete. References: PMID:33317024 Sources: GOC:cjm Definition: Inhibits the growth and recrystallization of ice crystals, thereby lowering the freezing point of water and preventing cellular damage at subzero temperatures. This activity is observed in various cold-adapted organisms, including certain fish, insects, and plants, and contributes to survival in extreme cold environments by stabilizing supercooled liquid states.